{
  "gene_symbol": "CRYBG2",
  "term_id": "UNKNOWN:0002",
  "gene": "UniProtKB:Q8N1P7",
  "gene_name": "Beta_gamma crystallin domain-containing protein 2",
  "term_label": "Unknown biological process"
}